{
  "gene": "UniProtKB:P09455",
  "gene_name": "Retinol-binding protein 1",
  "term_label": "fatty acid binding",
  "gene_symbol": "RBP1",
  "term_id": "GO:0005504"
}